IgZ immunoglobulin complex [GO:0071761] (cellular component) Definition: A protein complex composed of two identical immunoglobulin heavy chains of the IgZ isotype and two identical immunoglobulin light chains, held together by disulfide bonds. The IgZ isotype is also known as the IgT isotype in certain species of fish. Sources: GOC:add, ISBN:0781765196 Also known as: IgT immunoglobulin complex, IgT antibody, IgZ antibody Note: Note that an IgZ immunoglobulin complex has the function of antigen binding if a suitable antigen is available. Note that IgZ is found in bony fish, and called IgT in certain species, such as trout. Relationships: is a type of GO:0019814